positive regulation of erythrophore differentiation [GO:0048780] (biological process) Relationships: is a type of regulation of erythrophore differentiation [GO:0048778]; is a type of GO:0050942; positively regulates GO:0048773 Definition: Any process that activates or increases the frequency, rate or extent of erythrophore differentiation. Also known as: up regulation of erythrophore differentiation, up-regulation of erythrophore differentiation, upregulation of erythrophore differentiation, activation of erythrophore differentiation, stimulation of erythrophore differentiation Sources: GOC:mh